{
  "term_label": "phosphatidylserine binding",
  "gene": "UniProtKB:Q9BYG8",
  "gene_symbol": "GSDMC",
  "gene_name": "Gasdermin-C",
  "term_id": "GO:0001786"
}